{
  "term_label": "dynein intermediate chain binding",
  "gene_symbol": "DNHD1",
  "gene": "UniProtKB:Q96M86",
  "term_id": "GO:0045505",
  "gene_name": "Dynein heavy chain domain-containing protein 1"
}